{
  "term_id": "GO:0005886",
  "gene": "UniProtKB:P07550",
  "gene_symbol": "ADRB2",
  "gene_name": "Beta-2 adrenergic receptor",
  "term_label": "plasma membrane"
}